{
  "term_id": "UNKNOWN:0003",
  "gene_symbol": "MAGIX",
  "gene": "UniProtKB:Q9H6Y5",
  "gene_name": "PDZ domain-containing protein MAGIX",
  "term_label": "Unknown cellular component"
}